{
  "term_id": "GO:0005886",
  "gene": "UniProtKB:P39086",
  "gene_name": "Glutamate receptor ionotropic, kainate 1",
  "gene_symbol": "GRIK1",
  "term_label": "plasma membrane"
}